venom-mediated platelet aggregation [GO:0044478] (biological process) Sources: GOC:fj, GOC:jl Also known as: envenomation promoting platelet aggregation, envenomation resulting in positive regulation of platelet aggregation in another organism, envenomation resulting in positive regulation of platelet aggregation in other organism, venom-mediated platelet agglutination Relationships: is a type of venom-mediated blood coagulation [GO:0044469] Definition: A process in which an organism initiates, promotes, or enhances platelet aggregation in another organism via the action of a venom.